{
  "term_id": "UNKNOWN:0002",
  "term_label": "Unknown biological process",
  "gene": "UniProtKB:Q9NWT8",
  "gene_symbol": "AURKAIP1",
  "gene_name": "Small ribosomal subunit protein mS38"
}